{
  "term_label": "regulation of axonogenesis",
  "gene_symbol": "ARHGAP35",
  "term_id": "GO:0050770",
  "gene_name": "Rho GTPase-activating protein 35",
  "gene": "UniProtKB:Q9NRY4"
}